negative regulation of proline import across plasma membrane [GO:1902835] (biological process) Relationships: is a type of negative regulation of organic acid transport [GO:0032891]; is a type of GO:0034763; is a type of negative regulation of amino acid transport [GO:0051956]; is a type of regulation of proline import across plasma membrane [GO:1902834]; negatively regulates proline import across plasma membrane [GO:1905647] References: PMID:24344203 Sources: GOC:TermGenie, GO_REF:0000058 Subtypes: GO:1905736 Definition: Any process that stops, prevents or reduces the frequency, rate or extent of proline import into cell. Also known as: down regulation of proline import into cell, down-regulation of proline import into cell, downregulation of proline import into cell, negative regulation of proline import into cell, inhibition of proline import into cell